{
  "gene_symbol": "ARID3B",
  "term_id": "GO:0006357",
  "gene_name": "AT-rich interactive domain-containing protein 3B",
  "term_label": "regulation of transcription by RNA polymerase II",
  "gene": "UniProtKB:Q8IVW6"
}